{
  "gene_name": "Cadherin-4",
  "term_label": "catenin complex",
  "gene_symbol": "CDH4",
  "term_id": "GO:0016342",
  "gene": "UniProtKB:P55283"
}